{
  "gene_name": "Uncharacterized protein C2orf27A",
  "term_label": "Unknown molecular function",
  "gene_symbol": "C2orf27A",
  "gene": "UniProtKB:P0DPF5",
  "term_id": "UNKNOWN:0001"
}